{
  "gene_name": "Phosphotriesterase-related protein",
  "gene_symbol": "PTER",
  "term_id": "UNKNOWN:0002",
  "term_label": "Unknown biological process",
  "gene": "UniProtKB:Q96BW5"
}